{
  "term_label": "enoyl-CoA hydratase activity",
  "gene_symbol": "HADHA",
  "term_id": "GO:0004300",
  "gene": "UniProtKB:P40939",
  "gene_name": "Trifunctional enzyme subunit alpha, mitochondrial"
}